{
  "gene_symbol": "MEPCE",
  "gene_name": "7SK snRNA methylphosphate capping enzyme",
  "term_id": "GO:0040031",
  "gene": "UniProtKB:Q7L2J0",
  "term_label": "snRNA modification"
}